{
  "gene": "UniProtKB:Q9UPT8",
  "gene_symbol": "ZC3H4",
  "term_label": "negative regulation of DNA-templated transcription, elongation",
  "term_id": "GO:0032785",
  "gene_name": "Zinc finger CCCH domain-containing protein 4"
}